{
  "term_id": "GO:0042790",
  "gene_name": "Treacle protein",
  "term_label": "nucleolar large rRNA transcription by RNA polymerase I",
  "gene_symbol": "TCOF1",
  "gene": "UniProtKB:Q13428"
}